{
  "gene": "UniProtKB:P18084",
  "gene_name": "Integrin beta-5",
  "gene_symbol": "ITGB5",
  "term_id": "GO:0007160",
  "term_label": "cell-matrix adhesion"
}